adaptive immune response based on somatic recombination of immune receptors built from leucine-rich repeat domains [GO:0002459] (biological process) Definition: An immune response mediated by lymphocytes expressing specific receptors for antigen produced through a somatic diversification process that includes somatic recombination of variable lymphocyte receptors (VLR) incorporating leucine-rich repeat (LRR) domains, and allowing for enhanced responses upon subsequent exposures to the same antigen (immunological memory). Examples of this process are found in jawless fish, including the lampreys (Petromyzontidae) and hagfishes (Myxinidae). References: PMID:16373579 Sources: GOC:add, GOC:mtg_sensu Relationships: is a type of adaptive immune response [GO:0002250] Also known as: adaptive immune response based on somatic recombination of VLR built from LRR domains, adaptive immune response based on somatic recombination of variable lymphocyte receptors built from leucine-rich repeat domains, adaptive immune response in jawless fish